negative regulation of reductive pentose-phosphate cycle [GO:0080153] (biological process) Also known as: negative regulation of C3 photosynthesis, negative regulation of Calvin cycle Relationships: is_a negative regulation of biosynthetic process [GO:0009890]; is a type of negative regulation of carbohydrate metabolic process [GO:0045912]; is a type of regulation of reductive pentose-phosphate cycle [GO:0080152]; is a type of negative regulation of photosynthesis [GO:1905156]; negatively regulates reductive pentose-phosphate cycle [GO:0019253] References: PMID:17031544, PMID:20399532 Definition: Any process that stops, prevents, or reduces the frequency, rate or extent of the reductive pentose-phosphate cycle.